{
  "gene_symbol": "BGN",
  "term_label": "Unknown biological process",
  "gene": "UniProtKB:P21810",
  "gene_name": "Biglycan",
  "term_id": "UNKNOWN:0002"
}